{
  "term_id": "GO:0005768",
  "gene": "UniProtKB:Q8WXH6",
  "gene_name": "Ras-related protein Rab-40A",
  "gene_symbol": "RAB40A",
  "term_label": "endosome"
}